(+)-abscisic acid D-glucopyranosyl ester transmembrane transporter activity [GO:1902417] (molecular function) References: PMID:24028845 Sources: GOC:TermGenie Definition: Enables the transfer of (+)-abscisic acid D-glucopyranosyl ester from one side of a membrane to the other. Also known as: ABA-GE transmembrane transporter activity, abscisic acid glucosyl ester transmembrane transporter activity Relationships: is_a GO:0042947; is part of (+)-abscisic acid D-glucopyranosyl ester transmembrane transport [GO:1902418]